{
  "term_id": "UNKNOWN:0001",
  "gene_symbol": "CNOT10",
  "gene": "UniProtKB:Q9H9A5",
  "gene_name": "CCR4-NOT transcription complex subunit 10",
  "term_label": "Unknown molecular function"
}